{
  "term_label": "animal organ development",
  "gene_name": "Pro-neuregulin-2, membrane-bound isoform",
  "gene": "UniProtKB:O14511",
  "term_id": "GO:0048513",
  "gene_symbol": "NRG2"
}